{
  "term_id": "GO:0060828",
  "gene_name": "Cyclin N-terminal domain-containing protein",
  "gene": "UniProtKB:A0A8V8TMC4",
  "gene_symbol": "CCNYL1B",
  "term_label": "regulation of canonical Wnt signaling pathway"
}